{
  "gene": "UniProtKB:Q8WXS5",
  "gene_symbol": "CACNG8",
  "term_label": "channel regulator activity",
  "term_id": "GO:0016247",
  "gene_name": "Voltage-dependent calcium channel gamma-8 subunit"
}